formaldehyde dismutase activity [GO:0047895] (molecular function) Also known as: aldehyde dismutase activity, cannizzanase activity, formaldehyde:formaldehyde oxidoreductase activity, nicotinoprotein aldehyde dismutase Definition: Catalysis of the reaction: 2 formaldehyde + H2O = methanol + formate. Sources: EC:1.2.98.1 Relationships: is a type of oxidoreductase activity, acting on the aldehyde or oxo group of donors [GO:0016903]